{
  "term_id": "GO:0050862",
  "term_label": "positive regulation of T cell receptor signaling pathway",
  "gene_symbol": "CARD11",
  "gene": "UniProtKB:Q9BXL7",
  "gene_name": "Caspase recruitment domain-containing protein 11"
}